{
  "gene_name": "Peroxisome proliferator-activated receptor delta",
  "term_id": "GO:0000978",
  "term_label": "RNA polymerase II cis-regulatory region sequence-specific DNA binding",
  "gene_symbol": "PPARD",
  "gene": "UniProtKB:Q03181"
}